{
  "gene": "UniProtKB:A1XBS5",
  "term_id": "UNKNOWN:0001",
  "gene_symbol": "CIBAR1",
  "term_label": "Unknown molecular function",
  "gene_name": "CBY1-interacting BAR domain-containing protein 1"
}